{
  "term_id": "UNKNOWN:0002",
  "term_label": "Unknown biological process",
  "gene": "UniProtKB:P22532",
  "gene_symbol": "SPRR2D",
  "gene_name": "Small proline-rich protein 2D"
}